{
  "gene": "UniProtKB:P36894",
  "gene_symbol": "BMPR1A",
  "term_label": "BMP signaling pathway",
  "term_id": "GO:0030509",
  "gene_name": "Bone morphogenetic protein receptor type-1A"
}